{
  "term_label": "Unknown cellular component",
  "gene": "UniProtKB:P02745",
  "term_id": "UNKNOWN:0003",
  "gene_symbol": "C1QA",
  "gene_name": "Complement C1q subcomponent subunit A"
}